{
  "gene_symbol": "ZNF200",
  "gene_name": "Zinc finger protein 200",
  "term_id": "UNKNOWN:0003",
  "term_label": "Unknown cellular component",
  "gene": "UniProtKB:P98182"
}